{
  "gene_name": "Putative uncharacterized protein MGC15705",
  "term_id": "UNKNOWN:0001",
  "term_label": "Unknown molecular function",
  "gene": "UniProtKB:Q96IR3",
  "gene_symbol": "Q96IR3"
}